{
  "gene_name": "Insulin-like growth factor II",
  "term_label": "protein serine/threonine kinase activator activity",
  "term_id": "GO:0043539",
  "gene_symbol": "IGF2",
  "gene": "UniProtKB:P01344"
}